oxalate-CoA ligase activity [GO:0050203] (molecular function) Definition: Catalysis of the reaction: ATP + CoA + oxalate = AMP + diphosphate + H+ + oxalyl-CoA. Relationships: is a type of CoA-ligase activity [GO:0016405]; is a type of acid-thiol ligase activity [GO:0016878] Sources: RHEA:18293 Also known as: oxalate:CoA ligase (AMP-forming), oxalyl coenzyme A synthetase activity, oxalyl-CoA synthetase activity